{
  "term_label": "calcium channel activity",
  "gene_name": "Protein lifeguard 4",
  "gene_symbol": "TMBIM4",
  "term_id": "GO:0005262",
  "gene": "UniProtKB:Q9HC24"
}